{
  "term_label": "nucleus",
  "gene_symbol": "SFPQ",
  "term_id": "GO:0005634",
  "gene": "UniProtKB:P23246",
  "gene_name": "Splicing factor, proline- and glutamine-rich"
}